{
  "gene_symbol": "SERINC1",
  "term_label": "Unknown molecular function",
  "gene": "UniProtKB:Q9NRX5",
  "term_id": "UNKNOWN:0001",
  "gene_name": "Serine incorporator 1"
}